cell plate assembly [GO:0000919] (biological process) Relationships: is_a cell cycle process [GO:0022402]; is a type of cellular component assembly [GO:0022607]; BFO_0000050 cytokinesis by cell plate formation [GO:0000911] Subtypes: cell plate formation involved in plant-type cell wall biogenesis [GO:0009920] Also known as: cell plate formation Definition: The process of assembly, maturation, and growth of the cell plate to the cell periphery in cells that divide by cell plate formation; often involves deposition of cell wall material in and around the phragmoplast. Sources: GOC:clt